{
  "gene_symbol": "MEPCE",
  "term_id": "GO:0008173",
  "gene_name": "7SK snRNA methylphosphate capping enzyme",
  "gene": "UniProtKB:Q7L2J0",
  "term_label": "RNA methyltransferase activity"
}